{
  "term_label": "cell projection assembly",
  "gene_name": "Macrophage-capping protein",
  "gene": "UniProtKB:P40121",
  "term_id": "GO:0030031",
  "gene_symbol": "CAPG"
}